{
  "term_id": "GO:0050688",
  "gene_name": "ELMO domain-containing protein 2",
  "term_label": "regulation of defense response to virus",
  "gene": "UniProtKB:Q8IZ81",
  "gene_symbol": "ELMOD2"
}